common bile duct development [GO:0061009] (biological process) Relationships: is a type of tube development [GO:0035295]; is part of hepaticobiliary system development [GO:0061008] Also known as: EHBD development, extrahepatic bile duct development, CBD development, bile duct development Definition: The progression of the common bile duct over time, from its formation to the mature structure. The common bile duct is formed from the joining of the common hepatic duct running from the liver, and the cystic duct running from the gallbladder. The common bile duct transports bile from the liver and gallbladder to the intestine. References: PMID:20614624 Subtypes: GO:0035622, GO:0035628, hepatic duct development [GO:0061011]